{
  "term_label": "Unknown molecular function",
  "term_id": "UNKNOWN:0001",
  "gene_symbol": "GSAP",
  "gene": "UniProtKB:A4D1B5",
  "gene_name": "Gamma-secretase-activating protein"
}